{
  "term_label": "plasma membrane",
  "term_id": "GO:0005886",
  "gene_symbol": "MC5R",
  "gene": "UniProtKB:P33032",
  "gene_name": "Melanocortin receptor 5"
}